{
  "gene_name": "Olfactory receptor",
  "term_id": "GO:0007608",
  "gene_symbol": "OR5D3",
  "term_label": "sensory perception of smell",
  "gene": "UniProtKB:A0A2R8Y4L6"
}